{
  "gene_name": "Aurora kinase A",
  "term_label": "spindle midzone",
  "term_id": "GO:0051233",
  "gene_symbol": "AURKA",
  "gene": "UniProtKB:O14965"
}